{
  "term_label": "nucleus",
  "gene": "UniProtKB:P0CJ85",
  "gene_symbol": "DUX4L2",
  "term_id": "GO:0005634",
  "gene_name": "Double homeobox protein 4-like protein 2"
}